{
  "gene": "UniProtKB:O94929",
  "gene_name": "Actin-binding LIM protein 3",
  "term_label": "actin filament binding",
  "term_id": "GO:0051015",
  "gene_symbol": "ABLIM3"
}